{
  "term_id": "GO:0033564",
  "term_label": "anterior/posterior axon guidance",
  "gene_symbol": "UNC5B",
  "gene_name": "Netrin receptor UNC5B",
  "gene": "UniProtKB:Q8IZJ1"
}